{
  "gene_name": "Putative uncharacterized protein encoded by LINC00313",
  "gene_symbol": "LINC00313",
  "term_id": "UNKNOWN:0003",
  "gene": "UniProtKB:P59037",
  "term_label": "Unknown cellular component"
}